{
  "gene_name": "Mitochondrial peptide methionine sulfoxide reductase",
  "term_label": "cytoplasm",
  "gene": "UniProtKB:Q9UJ68",
  "gene_symbol": "MSRA",
  "term_id": "GO:0005737"
}